{
  "term_label": "Unknown biological process",
  "gene_symbol": "CCDC77",
  "gene": "UniProtKB:Q9BR77",
  "gene_name": "Coiled-coil domain-containing protein 77",
  "term_id": "UNKNOWN:0002"
}